{
  "term_id": "GO:0072659",
  "term_label": "protein localization to plasma membrane",
  "gene": "UniProtKB:Q12955",
  "gene_name": "Ankyrin-3",
  "gene_symbol": "ANK3"
}